{
  "gene_name": "Cytochrome P450 3A7",
  "term_id": "GO:0050649",
  "gene": "UniProtKB:P24462",
  "term_label": "testosterone 6-beta-hydroxylase activity",
  "gene_symbol": "CYP3A7"
}